{
  "gene_symbol": "RAB6B",
  "gene": "UniProtKB:Q9NRW1",
  "term_id": "GO:1903292",
  "term_label": "protein localization to Golgi membrane",
  "gene_name": "Ras-related protein Rab-6B"
}